{
  "gene": "UniProtKB:O96013",
  "gene_symbol": "PAK4",
  "gene_name": "Serine_threonine-protein kinase PAK 4",
  "term_label": "cytoplasm",
  "term_id": "GO:0005737"
}